{
  "term_label": "Unknown molecular function",
  "gene_symbol": "DEF8",
  "gene_name": "Differentially expressed in FDCP 8 homolog",
  "term_id": "UNKNOWN:0001",
  "gene": "UniProtKB:Q6ZN54"
}